{
  "gene_symbol": "PLXNC1",
  "gene_name": "Plexin-C1",
  "term_label": "regulation of cell shape",
  "gene": "UniProtKB:O60486",
  "term_id": "GO:0008360"
}